{
  "term_label": "positive regulation of transcription by RNA polymerase II",
  "gene": "UniProtKB:P23769",
  "gene_name": "Endothelial transcription factor GATA-2",
  "gene_symbol": "GATA2",
  "term_id": "GO:0045944"
}